{
  "gene": "UniProtKB:Q5TB80",
  "term_id": "GO:0005814",
  "term_label": "centriole",
  "gene_symbol": "CEP162",
  "gene_name": "Centrosomal protein of 162 kDa"
}